{
  "gene": "UniProtKB:O14994",
  "gene_symbol": "SYN3",
  "term_label": "synaptic vesicle clustering",
  "gene_name": "Synapsin-3",
  "term_id": "GO:0097091"
}